{
  "gene_symbol": "WDSUB1",
  "gene": "UniProtKB:Q8N9V3",
  "term_id": "UNKNOWN:0003",
  "term_label": "Unknown cellular component",
  "gene_name": "WD repeat, SAM and U-box domain-containing protein 1"
}